{
  "term_id": "GO:0034452",
  "term_label": "dynactin binding",
  "gene_name": "Protein bicaudal D homolog 1",
  "gene_symbol": "BICD1",
  "gene": "UniProtKB:Q96G01"
}